{
  "term_label": "5-phosphoribose 1-diphosphate biosynthetic process",
  "gene_name": "Phosphoribosyl pyrophosphate synthase-associated protein 1",
  "term_id": "GO:0006015",
  "gene": "UniProtKB:Q14558",
  "gene_symbol": "PRPSAP1"
}